{
  "gene_symbol": "GSTM2",
  "gene_name": "Glutathione S-transferase Mu 2",
  "term_id": "GO:0006749",
  "gene": "UniProtKB:P28161",
  "term_label": "glutathione metabolic process"
}